{
  "term_label": "RNA export from nucleus",
  "term_id": "GO:0006405",
  "gene": "UniProtKB:P37198",
  "gene_symbol": "NUP62",
  "gene_name": "Nuclear pore glycoprotein p62"
}